{
  "term_label": "cytosol",
  "gene_symbol": "AKR1C2",
  "term_id": "GO:0005829",
  "gene_name": "Aldo-keto reductase family 1 member C2",
  "gene": "UniProtKB:P52895"
}